{
  "gene": "UniProtKB:Q9Y6I3",
  "gene_name": "Epsin-1",
  "term_label": "clathrin vesicle coat",
  "gene_symbol": "EPN1",
  "term_id": "GO:0030125"
}